{
  "gene": "UniProtKB:Q8WUG5",
  "term_id": "UNKNOWN:0003",
  "gene_symbol": "SLC22A17",
  "gene_name": "Solute carrier family 22 member 17",
  "term_label": "Unknown cellular component"
}